{
  "gene_name": "Rho-related GTP-binding protein RhoB",
  "term_label": "actin filament organization",
  "term_id": "GO:0007015",
  "gene_symbol": "RHOB",
  "gene": "UniProtKB:P62745"
}